neurotransmitter receptor diffusion trapping [GO:0099628] (biological process) Subtypes: postsynaptic neurotransmitter receptor diffusion trapping [GO:0098970] Definition: The process by which diffusing neurotransmitter receptor becomes trapped in region of the plasma membrane. References: PMID:18832033 Relationships: is a type of receptor diffusion trapping [GO:0098953]; occurs in plasma membrane region [GO:0098590]